regulation of skeletal muscle hypertrophy [GO:1904204] (biological process) Relationships: is a type of GO:0014733; is a type of regulation of muscle hypertrophy [GO:0014743]; RO_0002211 skeletal muscle hypertrophy [GO:0014734] References: PMID:23470307 Sources: GOC:TermGenie, GO_REF:0000058 Subtypes: negative regulation of skeletal muscle hypertrophy [GO:1904205], positive regulation of skeletal muscle hypertrophy [GO:1904206] Definition: Any process that modulates the frequency, rate or extent of skeletal muscle hypertrophy.